{
  "gene_symbol": "ABCA1",
  "term_label": "phosphatidylcholine floppase activity",
  "term_id": "GO:0090554",
  "gene_name": "Phospholipid-transporting ATPase ABCA1",
  "gene": "UniProtKB:O95477"
}